{
  "gene_symbol": "GPR52",
  "term_label": "plasma membrane",
  "term_id": "GO:0005886",
  "gene_name": "G-protein coupled receptor 52",
  "gene": "UniProtKB:Q9Y2T5"
}